{
  "term_label": "negative regulation of regulatory ncRNA-mediated heterochromatin formation",
  "gene_symbol": "ERI3",
  "gene_name": "ERI1 exoribonuclease 3",
  "term_id": "GO:0060906",
  "gene": "UniProtKB:O43414"
}